{
  "gene_symbol": "KCNN1",
  "gene": "UniProtKB:Q92952",
  "term_id": "GO:0043025",
  "gene_name": "Small conductance calcium-activated potassium channel protein 1",
  "term_label": "neuronal cell body"
}